{
  "gene": "UniProtKB:A0A0C4DH26",
  "term_label": "immunoglobulin complex",
  "gene_name": "Probable non-functional immunoglobulin kappa variable 6D-41",
  "gene_symbol": "IGKV6D-41",
  "term_id": "GO:0019814"
}